{
  "gene_symbol": "TRPC6",
  "term_id": "GO:0005886",
  "gene": "UniProtKB:Q9Y210",
  "gene_name": "Short transient receptor potential channel 6",
  "term_label": "plasma membrane"
}